protein phosphatase type 2A complex [GO:0000159] (cellular component) References: PMID:17245430 Sources: GOC:mah, ISBN:0198547684 Definition: A protein complex that has protein serine/threonine phosphatase activity that is polycation-stimulated (PCS), being directly stimulated by protamine, polylysine, or histone H1; it constitutes a subclass of several enzymes activated by different histones and polylysine, and consists of catalytic, scaffolding, and regulatory subunits. The catalytic and scaffolding subunits form the core enzyme, and the holoenzyme also includes the regulatory subunit. Also known as: PP2A complex, PP2A-pi, PP2a-protector, protein phosphatase 2 complex Relationships: is a type of protein serine/threonine phosphatase complex [GO:0008287]